{
  "gene_name": "Cytoplasmic protein NCK1",
  "gene_symbol": "NCK1",
  "term_id": "GO:1903898",
  "term_label": "negative regulation of PERK-mediated unfolded protein response",
  "gene": "UniProtKB:P16333"
}